{
  "term_id": "GO:0072542",
  "term_label": "protein phosphatase activator activity",
  "gene": "UniProtKB:Q13362",
  "gene_symbol": "PPP2R5C",
  "gene_name": "Serine_threonine-protein phosphatase 2A 56 kDa regulatory subunit gamma isoform"
}